{
  "gene_symbol": "MYH15",
  "term_id": "GO:0005737",
  "gene_name": "Myosin-15",
  "term_label": "cytoplasm",
  "gene": "UniProtKB:Q9Y2K3"
}